{
  "gene": "UniProtKB:Q14934",
  "term_label": "RNA polymerase II cis-regulatory region sequence-specific DNA binding",
  "gene_name": "Nuclear factor of activated T-cells, cytoplasmic 4",
  "gene_symbol": "NFATC4",
  "term_id": "GO:0000978"
}